{
  "gene": "UniProtKB:O75533",
  "gene_symbol": "SF3B1",
  "gene_name": "Splicing factor 3B subunit 1",
  "term_label": "U2-type prespliceosome",
  "term_id": "GO:0071004"
}